{
  "gene_symbol": "CATSPERG",
  "term_id": "GO:0036128",
  "gene": "UniProtKB:Q6ZRH7",
  "gene_name": "Cation channel sperm-associated auxiliary subunit gamma",
  "term_label": "CatSper complex"
}